positive regulation of transport [GO:0051050] (BP) Definition: Any process that activates or increases the frequency, rate or extent of the directed movement of substances (such as macromolecules, small molecules, ions) into, out of or within a cell, or between cells, by means of some agent such as a transporter or pore. Relationships: is a type of positive regulation of biological process [GO:0048518]; is a type of regulation of transport [GO:0051049]; positively regulates transport [GO:0006810] Sources: GOC:ai Subtypes: GO:0031340, GO:0032241, positive regulation of lipid transport [GO:0032370], positive regulation of intracellular transport [GO:0032388], positive regulation of transporter activity [GO:0032411], GO:0032892, positive regulation of transmembrane transport [GO:0034764], GO:0035540, positive regulation of monoatomic ion transport [GO:0043270], positive regulation of endocytosis [GO:0045807], positive regulation of secretion [GO:0051047], positive regulation of protein transport [GO:0051222], positive regulation of neurotransmitter transport [GO:0051590], positive regulation of norepinephrine uptake [GO:0051623], positive regulation of epinephrine uptake [GO:0051628], positive regulation of amine transport [GO:0051954], GO:0150201, positive regulation of cellotriose transport [GO:1900287], positive regulation of galactotriose transport [GO:1900293], positive regulation of heptasaccharide transport [GO:1900296], positive regulation of hexasaccharide transport [GO:1900299], positive regulation of laminaritriose transport [GO:1900305], GO:1900323, positive regulation of maltotriulose transport [GO:1900326], positive regulation of mannotriose transport [GO:1900329], GO:1900359, positive regulation of pentasaccharide transport [GO:1900362], GO:1901030, positive regulation of peptide antigen transport [GO:1901041], positive regulation of maltose transport [GO:1902345], positive regulation of synaptic vesicle transport [GO:1902805], positive regulation of melanosome transport [GO:1902910], GO:1903423, positive regulation of transcytosis [GO:1904300], GO:1905367, positive regulation of sodium-dependent phosphate transport [GO:2000120], GO:2000809, GO:2000878, positive regulation of renal water transport [GO:2001153] Also known as: up regulation of transport, up-regulation of transport, upregulation of transport, activation of transport, stimulation of transport